fungal-type cell wall (1->3)-beta-D-glucan biosynthetic process [GO:0071970] (biological process) Definition: The chemical reactions and pathways resulting in the formation of (1->3)-beta-D-glucans, compounds composed of glucose residues linked by (1->3)-beta-D-glucosidic bonds, found in fungal cell walls. Sources: GOC:mah Also known as: fungal-type cell wall 1,3-beta-D-glucan biosynthetic process, fungal-type cell wall 1,3-beta-glucan anabolism, fungal-type cell wall 1,3-beta-glucan biosynthesis, fungal-type cell wall 1,3-beta-glucan formation, fungal-type cell wall 1,3-beta-glucan synthesis, fungal-type cell wall beta-1,3-glucan anabolism, fungal-type cell wall beta-1,3-glucan biosynthesis, fungal-type cell wall beta-1,3-glucan biosynthetic process, fungal-type cell wall beta-1,3-glucan formation, fungal-type cell wall beta-1,3-glucan synthesis Relationships: is a type of cell wall (1->3)-beta-D-glucan biosynthetic process [GO:0034411]; is a type of GO:0070880; is a type of fungal-type cell wall (1->3)-beta-D-glucan metabolic process [GO:0071969] Subtypes: ascospore wall (1->3)-beta-D-glucan biosynthetic process [GO:0034413]